{
  "term_id": "UNKNOWN:0001",
  "gene": "UniProtKB:Q8IZT9",
  "term_label": "Unknown molecular function",
  "gene_symbol": "FAM9C",
  "gene_name": "Protein FAM9C"
}